{
  "term_id": "GO:0070588",
  "gene": "UniProtKB:P48995",
  "term_label": "calcium ion transmembrane transport",
  "gene_name": "Short transient receptor potential channel 1",
  "gene_symbol": "TRPC1"
}